D-loop DNA binding [GO:0062037] (molecular function) Subtypes: telomeric D-loop binding [GO:0061821] Relationships: is a type of DNA secondary structure binding [GO:0000217] Also known as: DNA displacement loop binding References: PMID:20924116 Definition: Binding to a DNA D-loop. A D-loop is a three-stranded DNA structure formed by the invasion of a single DNA strand that base pairs with one strand of duplex DNA, while the rest of the double-stranded DNA does not unwind.